{
  "gene_name": "Cilia- and flagella-associated protein 299",
  "term_label": "Unknown molecular function",
  "term_id": "UNKNOWN:0001",
  "gene": "UniProtKB:Q6V702",
  "gene_symbol": "CFAP299"
}